{
  "term_id": "GO:0034198",
  "gene_name": "GATOR complex protein MIOS",
  "term_label": "cellular response to amino acid starvation",
  "gene_symbol": "MIOS",
  "gene": "UniProtKB:Q9NXC5"
}